{
  "term_label": "mitochondrion",
  "term_id": "GO:0005739",
  "gene_symbol": "MTHFS",
  "gene": "UniProtKB:P49914",
  "gene_name": "5-formyltetrahydrofolate cyclo-ligase"
}